{
  "gene_name": "Transcription factor MafF",
  "gene": "UniProtKB:Q9ULX9",
  "term_id": "GO:0000981",
  "gene_symbol": "MAFF",
  "term_label": "DNA-binding transcription factor activity, RNA polymerase II-specific"
}